{
  "term_id": "GO:0004708",
  "term_label": "MAP kinase kinase activity",
  "gene_symbol": "SBK2",
  "gene_name": "Serine_threonine-protein kinase SBK2",
  "gene": "UniProtKB:P0C263"
}